{
  "gene_name": "SWI_SNF complex subunit SMARCC2",
  "gene": "UniProtKB:Q8TAQ2",
  "term_label": "positive regulation of DNA-templated transcription",
  "term_id": "GO:0045893",
  "gene_symbol": "SMARCC2"
}